{
  "gene_symbol": "TAFA5",
  "term_id": "GO:0005615",
  "gene": "UniProtKB:Q7Z5A7",
  "gene_name": "Chemokine-like protein TAFA-5",
  "term_label": "extracellular space"
}